{
  "gene_symbol": "FSCN3",
  "gene_name": "Fascin-3",
  "term_label": "filopodium",
  "term_id": "GO:0030175",
  "gene": "UniProtKB:Q9NQT6"
}